{
  "gene": "UniProtKB:P25098",
  "term_label": "G protein-coupled receptor signaling pathway",
  "term_id": "GO:0007186",
  "gene_name": "Beta-adrenergic receptor kinase 1",
  "gene_symbol": "GRK2"
}